{
  "gene": "UniProtKB:P83111",
  "gene_name": "Serine beta-lactamase-like protein LACTB, mitochondrial",
  "term_id": "GO:0005739",
  "term_label": "mitochondrion",
  "gene_symbol": "LACTB"
}